{
  "gene_symbol": "FGF8",
  "term_id": "GO:0030334",
  "gene_name": "Fibroblast growth factor 8",
  "gene": "UniProtKB:P55075",
  "term_label": "regulation of cell migration"
}